{
  "term_id": "GO:1990834",
  "term_label": "response to odorant",
  "gene": "UniProtKB:A5D8W1",
  "gene_symbol": "CFAP69",
  "gene_name": "Cilia- and flagella-associated protein 69"
}